{
  "gene": "UniProtKB:Q9BRQ0",
  "term_label": "Unknown molecular function",
  "term_id": "UNKNOWN:0001",
  "gene_symbol": "PYGO2",
  "gene_name": "Pygopus homolog 2"
}